{
  "gene_name": "ATP-binding cassette sub-family D member 1",
  "gene_symbol": "ABCD1",
  "term_label": "peroxisomal membrane",
  "gene": "UniProtKB:P33897",
  "term_id": "GO:0005778"
}